central T cell tolerance induction [GO:0002512] (biological process) Also known as: central T lymphocyte tolerance induction, central T-cell tolerance induction, central T-lymphocyte tolerance induction Definition: Tolerance induction of T cells in the thymus. Sources: GOC:jal, ISBN:0781735149 Relationships: is a type of central tolerance induction [GO:0002508]; is a type of T cell tolerance induction [GO:0002517]